nucleus organization [GO:0006997] (BP) Sources: GOC:dph, GOC:ems, GOC:jl, GOC:mah Definition: A process that is carried out at the cellular level which results in the assembly, arrangement of constituent parts, or disassembly of the nucleus. Regulation: regulated by regulation of nucleus organization [GO:1903353] Relationships: is a type of organelle organization [GO:0006996] Also known as: nuclear organisation, nuclear organization, nuclear morphology, nuclear organization and biogenesis, nucleus organization and biogenesis Subtypes: karyogamy [GO:0000741], nuclear pore organization [GO:0006999], nucleolus organization [GO:0007000], GO:0007289, spermatid nucleus elongation [GO:0007290], nuclear body organization [GO:0030575], macronucleus organization [GO:0032124], GO:0032125, GO:0035038, male pronucleus assembly [GO:0035039], nuclear matrix organization [GO:0043578], nuclear pore localization [GO:0051664], GO:1905690